{
  "gene_name": "KH domain-containing protein 3",
  "term_label": "Unknown molecular function",
  "gene_symbol": "KHDC3L",
  "gene": "UniProtKB:Q587J8",
  "term_id": "UNKNOWN:0001"
}